{
  "term_id": "GO:0016887",
  "term_label": "ATP hydrolysis activity",
  "gene": "UniProtKB:Q96L93",
  "gene_symbol": "KIF16B",
  "gene_name": "Kinesin-like protein KIF16B"
}